{
  "term_label": "Unknown cellular component",
  "gene": "UniProtKB:P78363",
  "gene_symbol": "ABCA4",
  "gene_name": "Retinal-specific phospholipid-transporting ATPase ABCA4",
  "term_id": "UNKNOWN:0003"
}